{
  "gene_symbol": "HES4",
  "gene_name": "Transcription factor HES-4",
  "term_id": "GO:0005634",
  "term_label": "nucleus",
  "gene": "UniProtKB:Q9HCC6"
}